{
  "gene_name": "Immunoglobulin heavy constant epsilon",
  "gene_symbol": "IGHE",
  "term_label": "immunoglobulin complex, circulating",
  "term_id": "GO:0042571",
  "gene": "UniProtKB:P01854"
}